{
  "gene_symbol": "JUNB",
  "term_id": "GO:0045944",
  "gene": "UniProtKB:P17275",
  "term_label": "positive regulation of transcription by RNA polymerase II",
  "gene_name": "Transcription factor JunB"
}